{
  "term_label": "negative regulation of transcription by RNA polymerase II",
  "gene_name": "Homeobox protein TGIF2",
  "gene_symbol": "TGIF2",
  "term_id": "GO:0000122",
  "gene": "UniProtKB:Q9GZN2"
}